{
  "gene": "UniProtKB:P17693",
  "gene_symbol": "HLA-G",
  "gene_name": "HLA class I histocompatibility antigen, alpha chain G",
  "term_id": "GO:0030881",
  "term_label": "beta-2-microglobulin binding"
}